{
  "gene_symbol": "NUCB2",
  "gene_name": "Nucleobindin-2",
  "term_label": "Unknown biological process",
  "term_id": "UNKNOWN:0002",
  "gene": "UniProtKB:P80303"
}